telomeric loop formation [GO:0031627] (biological process) Definition: The process in which linear telomeric DNA is remodeled into duplex loops, by the invasion of a 3' single-stranded overhang into the duplex region. References: PMID:10338214 Sources: GOC:vw Also known as: T loop biosynthesis, T loop formation, t-loop biosynthesis, t-loop formation Relationships: is a type of telomere maintenance [GO:0000723] Regulation: regulated by regulation of telomeric loop formation [GO:1904418]; negatively regulated by negative regulation of telomeric loop formation [GO:1904419]; positively regulated by GO:1904420